glycosaminoglycan-protein linkage region biosynthetic process [GO:0120532] (biological process) Definition: The formation of a tetrasaccharide linker sequence (xylose-galactose-galactose-glucuronate) on specific serine residues of a core protein, on to which dermatan sulfate, chondroitin sulfate, heparan sulfate or heparin glycosaminoglycans may be assembled to synthesise the corresponding proteoglycan. Sources: MetaCyc:PWY-6557 Also known as: Glycosaminoglycan biosynthesis, linkage tetrasaccharide, glycosaminoglycan-protein linkage region biosynthesis Relationships: is a type of protein O-linked glycosylation via xylose [GO:0180064]; BFO_0000050 GO:0015012; is part of GO:0030210; BFO_0000050 chondroitin sulfate proteoglycan biosynthetic process [GO:0050650]; is part of GO:0050651